nucleobase binding [GO:0002054] (molecular function) Sources: GOC:hjd Subtypes: purine nucleobase binding [GO:0002060], GO:0002061 Relationships: is a type of heterocyclic compound binding [GO:1901363] Definition: Binding to a nucleobase, any of a class of pyrmidines or purines, organic nitrogenous bases.